cytoneme assembly [GO:0035231] (biological process) Also known as: cytoneme biogenesis Definition: Formation of a cytoneme, a long, thin and polarized actin-based cytoplasmic extension that projects from a cell. References: PMID:10367889, PMID:10675901 Relationships: is a type of cellular component assembly involved in morphogenesis [GO:0010927]; is a type of GO:0120031; is part of cytoneme morphogenesis [GO:0003399]